response to proline [GO:0010238] (biological process) Subtypes: GO:0071235 Definition: Any process that results in a change in state or activity of a cell or an organism (in terms of movement, secretion, enzyme production, gene expression, etc.) as a result of a proline stimulus. Sources: GOC:sm Relationships: is a type of response to amino acid [GO:0043200]; is_a response to nitrogen compound [GO:1901698]; is a type of GO:1901700